{
  "gene_name": "Putative ankyrin repeat domain-containing protein 20A2",
  "term_id": "UNKNOWN:0003",
  "term_label": "Unknown cellular component",
  "gene": "UniProtKB:Q5SQ80",
  "gene_symbol": "ANKRD20A2P"
}